{
  "term_id": "GO:0043524",
  "gene": "UniProtKB:Q9BWQ8",
  "term_label": "negative regulation of neuron apoptotic process",
  "gene_symbol": "FAIM2",
  "gene_name": "Protein lifeguard 2"
}